{
  "term_label": "recycling endosome",
  "gene_name": "WAS protein family homolog 6",
  "term_id": "GO:0055037",
  "gene_symbol": "WASH6P",
  "gene": "UniProtKB:Q9NQA3"
}